{
  "gene": "UniProtKB:P04000",
  "term_label": "plasma membrane",
  "term_id": "GO:0005886",
  "gene_name": "Long-wave-sensitive opsin 1",
  "gene_symbol": "OPN1LW"
}